{
  "gene_symbol": "MICAL1",
  "term_id": "GO:0051015",
  "gene": "UniProtKB:Q8TDZ2",
  "gene_name": "[F-actin]-monooxygenase MICAL1",
  "term_label": "actin filament binding"
}